{
  "gene_name": "Large ribosomal subunit protein mL38",
  "term_id": "UNKNOWN:0002",
  "gene_symbol": "MRPL38",
  "term_label": "Unknown biological process",
  "gene": "UniProtKB:Q96DV4"
}